{
  "term_label": "voltage-gated chloride channel activity",
  "gene_symbol": "CLCN1",
  "gene_name": "Chloride channel protein 1",
  "term_id": "GO:0005247",
  "gene": "UniProtKB:P35523"
}